response to brefeldin A [GO:0031001] (biological process) Relationships: is a type of response to antibiotic [GO:0046677]; is a type of GO:1901700 Subtypes: cellular response to brefeldin A [GO:0071238] Sources: GOC:mah Definition: Any process that results in a change in state or activity of a cell or an organism (in terms of movement, secretion, enzyme production, gene expression, etc.) as a result of a brefeldin A stimulus.